{
  "gene_symbol": "BLOC1S2",
  "gene_name": "Biogenesis of lysosome-related organelles complex 1 subunit 2",
  "term_label": "BLOC-1 complex",
  "gene": "UniProtKB:Q6QNY1",
  "term_id": "GO:0031083"
}